{
  "gene_name": "Solute carrier family 25 member 43",
  "gene": "UniProtKB:Q8WUT9",
  "term_id": "UNKNOWN:0002",
  "gene_symbol": "SLC25A43",
  "term_label": "Unknown biological process"
}